{
  "gene": "UniProtKB:P22310",
  "term_label": "UDP-glycosyltransferase activity",
  "term_id": "GO:0008194",
  "gene_symbol": "UGT1A4",
  "gene_name": "UDP-glucuronosyltransferase 1A4"
}